L-leucine import across plasma membrane [GO:1903801] (biological process) Also known as: L-leucine import, leucine import, L-leucine import into cell, leucine uptake, L-leucine uptake References: PMID:23895341 Sources: GOC:TermGenie, GO_REF:0000075 Regulation: regulated by regulation of L-leucine import across plasma membrane [GO:1905532]; negatively regulated by negative regulation of L-leucine import across plasma membrane [GO:1905533]; positively regulated by positive regulation of L-leucine import across plasma membrane [GO:1905534] Relationships: is a type of L-leucine transport [GO:0015820]; is a type of amino acid import across plasma membrane [GO:0089718]; is a type of L-alpha-amino acid transmembrane transport [GO:1902475] Definition: The directed movement of L-leucine from outside of a cell, across the plasma membrane and into the cytosol.